{
  "term_label": "synaptic vesicle budding from presynaptic endocytic zone membrane",
  "gene_name": "Interferon-induced GTP-binding protein Mx1",
  "term_id": "GO:0016185",
  "gene_symbol": "MX1",
  "gene": "UniProtKB:P20591"
}